juxtaglomerulus cell development [GO:0072142] (BP) Definition: The process whose specific outcome is the progression of a juxtaglomerulus cell over time, from its formation to the mature structure. Sources: GOC:mtg_kidney_jan10 Subtypes: mesonephric juxtaglomerulus cell development [GO:0061229], metanephric juxtaglomerulus cell development [GO:0072252] Relationships: is a type of GO:0048468; is part of GO:0072052